{
  "term_label": "late endosome membrane",
  "gene_symbol": "HLA-DMA",
  "term_id": "GO:0031902",
  "gene": "UniProtKB:P28067",
  "gene_name": "HLA class II histocompatibility antigen, DM alpha chain"
}